phospholipase C-activating tachykinin receptor signaling pathway [GO:0007209] (BP) Sources: GOC:dph, GOC:mah, GOC:signaling, GOC:tb Relationships: is a type of phospholipase C-activating G protein-coupled receptor signaling pathway [GO:0007200]; is a type of tachykinin receptor signaling pathway [GO:0007217] Also known as: activation of phospholipase C activity by tachykinin receptor signaling pathway, activation of phospholipase C activity by tachykinin receptor signalling pathway, tachykinin receptor, phospholipase C activating pathway Definition: A phospholipase C-activating receptor G protein-coupled receptor signaling pathway initiated by tachykinin binding to its receptor on the surface of a target cell, and ending with the regulation of a downstream cellular process, e.g. transcription.